spatial regulation of meiotic DNA double-strand break formation involved in reciprocal meiotic recombination [GO:0062209] (biological process) Also known as: regulation of spatial distribution of meiotic DNA double-strand break formation involved in reciprocal meiotic recombination, regulation of spatial distribution of meiotic DSB formation involved in reciprocal meiotic recombination, DSB interference, crossover interference Relationships: is a type of GO:1905261 References: PMID:25324213, PMID:30217891 Definition: Any process that modulates the distribution of sites along the chromosome where meiotic DNA double-strand break formation takes place as part of reciprocal meiotic recombination.